{
  "term_id": "UNKNOWN:0002",
  "gene_symbol": "FAM169BP",
  "gene_name": "Protein FAM169BP",
  "term_label": "Unknown biological process",
  "gene": "UniProtKB:Q8N8A8"
}